{
  "term_id": "GO:0000398",
  "gene_symbol": "SF3B2",
  "gene": "UniProtKB:Q13435",
  "term_label": "mRNA splicing, via spliceosome",
  "gene_name": "Splicing factor 3B subunit 2"
}